{
  "gene_symbol": "MEIS1",
  "gene": "UniProtKB:O00470",
  "term_label": "positive regulation of transcription by RNA polymerase II",
  "gene_name": "Homeobox protein Meis1",
  "term_id": "GO:0045944"
}